acetylcholine transmembrane transporter activity [GO:0005277] (molecular function) Definition: Enables the transfer of acetylcholine from one side of a membrane to the other. Acetylcholine is an acetic acid ester of the organic base choline and functions as a neurotransmitter, released at the synapses of parasympathetic nerves and at neuromuscular junctions. Subtypes: acetylcholine:proton antiporter activity [GO:0005278] Sources: GOC:ai Relationships: is_a neurotransmitter transmembrane transporter activity [GO:0005326]; is_a acetate ester transmembrane transporter activity [GO:1901375]